malate dehydrogenase (decarboxylating) (NADP+) activity [GO:0004473] (molecular function) Definition: Catalysis of the reaction: (S)-malate + NADP+ = pyruvate + CO2 + NADPH. Relationships: is a type of GO:0004470; is_a oxidoreductase activity, acting on the CH-OH group of donors, NAD or NADP as acceptor [GO:0016616] Sources: RHEA:18253 Also known as: 'malic' enzyme, (S)-malate:NADP+ oxidoreductase (oxaloacetate-decarboxylating), L-malate:NADP oxidoreductase activity, NADP-linked decarboxylating malic enzyme, NADP-malic enzyme activity, NADP-specific malate dehydrogenase activity, NADP-specific malic enzyme, malate dehydrogenase (NADP, decarboxylating), malate dehydrogenase (decarboxylating, NADP) Note: For decarboxylation of oxaloacetate (the second substrate listed in EC:1.1.1.40), see 'oxaloacetate decarboxylase activity ; GO:0008948'.